{
  "gene": "UniProtKB:P61006",
  "term_label": "endocytic recycling",
  "gene_name": "Ras-related protein Rab-8A",
  "term_id": "GO:0032456",
  "gene_symbol": "RAB8A"
}